{
  "term_id": "GO:0051119",
  "gene": "UniProtKB:Q9BRV3",
  "term_label": "sugar transmembrane transporter activity",
  "gene_name": "Sugar transporter SWEET1",
  "gene_symbol": "SLC50A1"
}